organic phosphonate biosynthetic process [GO:0032923] (biological process) Also known as: organophosphonate biosynthetic process Definition: The chemical reactions and pathways resulting in the formation of phosphonates, any organic compound containing one or more C-PO(OH)2 or C-PO(OR)2 (with R=alkyl, aryl) groups. Synthesis of phosphonic acid itself, an inorganic compound without the biochemically relevant C-P bond, is not included. Sources: GOC:js Relationships: is a type of biosynthetic process [GO:0009058]; is a type of organic phosphonate metabolic process [GO:0019634]